{
  "term_label": "intracellular protein transport",
  "gene_symbol": "ARF3",
  "gene_name": "ADP-ribosylation factor 3",
  "gene": "UniProtKB:P61204",
  "term_id": "GO:0006886"
}